anion binding [GO:0043168] (molecular function) Subtypes: GO:0000822, phosphatidylserine binding [GO:0001786], UTP binding [GO:0002134], GO:0002135, phosphatidylinositol-4,5-bisphosphate binding [GO:0005546], GO:0005547, FMN binding [GO:0010181], AMP binding [GO:0016208], GMP binding [GO:0019002], GDP binding [GO:0019003], pyridoxal phosphate binding [GO:0030170], cAMP binding [GO:0030552], cGMP binding [GO:0030553], GO:0030973, thiamine pyrophosphate binding [GO:0030976], chloride ion binding [GO:0031404], carboxylic acid binding [GO:0031406], dAMP binding [GO:0032562], dADP binding [GO:0032563], dATP binding [GO:0032564], dGMP binding [GO:0032565], GO:0032566, dGTP binding [GO:0032567], ethanol binding [GO:0035276], cyclic-di-GMP binding [GO:0035438], purine ribonucleoside triphosphate binding [GO:0035639], lysophosphatidic acid binding [GO:0035727], S-nitrosoglutathione binding [GO:0035730], thiosulfate binding [GO:0036173], phosphate ion binding [GO:0042301], sulfate binding [GO:0043199], GO:0043210, glutathione binding [GO:0043295], phosphatidylinositol-3,4-bisphosphate binding [GO:0043325], ADP binding [GO:0043531], inositol 1,3,4,5 tetrakisphosphate binding [GO:0043533], suramin binding [GO:0043924], GO:0046714, 3'-phosphoadenosine 5'-phosphosulfate binding [GO:0050656], GO:0050660, 2',3'-cyclic GMP-AMP binding [GO:0061507], fructose-6-phosphate binding [GO:0070095], phosphatidic acid binding [GO:0070300], GO:0070401, NADPH binding [GO:0070402], NAD+ binding [GO:0070403], NADH binding [GO:0070404], inositol 1,4,5 trisphosphate binding [GO:0070679], bicarbonate binding [GO:0071890], GO:0072570, phosphatidylinositol-3,5-bisphosphate binding [GO:0080025], guanosine tetraphosphate binding [GO:0097216], GO:0097244, coenzyme A binding [GO:0120225], acyl-CoA binding [GO:0120227], prenyl-FMNH2 binding [GO:0120233], 3',3'-cyclic GMP-AMP binding [GO:0140703], 3',2'-cyclic GMP-AMP binding [GO:0140704], GO:1901359, hypochlorite binding [GO:1901531], GO:1901611, 5-O-phosphono-alpha-D-ribofuranosyl diphosphate binding [GO:1902248], GO:1902249, ceramide 1-phosphate binding [GO:1902387], riboflavin binding [GO:1902444], GO:1902516, enterobactin binding [GO:1903981], GO:1904492, quercitrin binding [GO:2001227] Definition: Binding to an anion, a charged atom or group of atoms with a net negative charge. Relationships: is a type of ion binding [GO:0043167] Sources: GOC:jl